{
  "gene_symbol": "TACC3",
  "gene_name": "Transforming acidic coiled-coil-containing protein 3",
  "term_label": "nuclear migration",
  "term_id": "GO:0007097",
  "gene": "UniProtKB:Q9Y6A5"
}